{
  "term_label": "SCF complex assembly",
  "term_id": "GO:0010265",
  "gene_name": "Cullin-associated NEDD8-dissociated protein 2",
  "gene": "UniProtKB:O75155",
  "gene_symbol": "CAND2"
}